{
  "term_id": "GO:0034315",
  "gene_name": "Arfaptin-2",
  "gene_symbol": "ARFIP2",
  "gene": "UniProtKB:P53365",
  "term_label": "regulation of Arp2/3 complex-mediated actin nucleation"
}